{
  "gene": "UniProtKB:P26441",
  "gene_symbol": "CNTF",
  "term_id": "GO:0030424",
  "term_label": "axon",
  "gene_name": "Ciliary neurotrophic factor"
}